{
  "term_label": "stress fiber",
  "gene_symbol": "PDLIM4",
  "gene": "UniProtKB:P50479",
  "gene_name": "PDZ and LIM domain protein 4",
  "term_id": "GO:0001725"
}